{
  "gene_symbol": "HSFX3",
  "gene_name": "Heat shock transcription factor, X-linked member 3",
  "gene": "UniProtKB:A0A1B0GWH4",
  "term_label": "Unknown biological process",
  "term_id": "UNKNOWN:0002"
}